{
  "term_label": "Unknown molecular function",
  "gene_name": "Putative uncharacterized protein C1orf220",
  "gene_symbol": "C1orf220",
  "term_id": "UNKNOWN:0001",
  "gene": "UniProtKB:Q5T0J3"
}